{
  "term_label": "apical plasma membrane",
  "gene": "UniProtKB:Q8TF72",
  "term_id": "GO:0016324",
  "gene_symbol": "SHROOM3",
  "gene_name": "Protein Shroom3"
}